acetyl-CoA assimilation pathway [GO:0019681] (biological process) Definition: The pathways by which acetyl-CoA is processed and converted into alpha-ketoglutarate (2-oxoglutarate); methanogenic archaea use these pathways to assimilate acetyl-CoA into the cell. Sources: MetaCyc:P22-PWY Also known as: acetyl-CoA catabolic process to 2-ketoglutarate, acetyl-CoA catabolic process to 2-oxoglutarate, acetyl-CoA catabolic process to alpha-ketoglutarate, acetyl-CoA catabolic process to alpha-oxoglutarate, acetyl-CoA catabolism to 2-ketoglutarate, acetyl-CoA catabolism to 2-oxoglutarate, acetyl-CoA catabolism to alpha-ketoglutarate, acetyl-CoA catabolism to alpha-oxoglutarate Relationships: is a type of 2-oxoglutarate metabolic process [GO:0006103]; is a type of acetyl-CoA catabolic process [GO:0046356]